{
  "term_label": "chromosome",
  "term_id": "GO:0005694",
  "gene": "UniProtKB:Q15645",
  "gene_symbol": "TRIP13",
  "gene_name": "Pachytene checkpoint protein 2 homolog"
}